L-proline import across plasma membrane [GO:1904271] (biological process) Regulation: regulated by regulation of L-proline import across plasma membrane [GO:1905735]; negatively regulated by GO:1905736; positively regulated by GO:1905737 Relationships: is_a L-proline transmembrane transport [GO:1904555]; is a type of proline import across plasma membrane [GO:1905647] Also known as: L-proline import into cell Definition: The directed movement of L-proline from outside of a cell, across the plasma membrane and into the cytosol. References: PMID:21097500 Sources: GOC:TermGenie, GOC:kmv, GO_REF:0000075